dynamic microtubule bundle [GO:0099071] (cellular component) Definition: A microtubule bundle that undergoes changes in length, and in which microtubule sliding takes place. Relationships: is a type of microtubule bundle [GO:0097427] References: PMID:26124291 Sources: GOC:vw